{
  "gene_name": "WASP homolog-associated protein with actin, membranes and microtubules",
  "term_id": "GO:0033116",
  "gene": "UniProtKB:Q8TF30",
  "gene_symbol": "WHAMM",
  "term_label": "endoplasmic reticulum-Golgi intermediate compartment membrane"
}